actinin binding [GO:0042805] (molecular function) Definition: Binding to actinin, any member of a family of proteins that crosslink F-actin. Sources: GOC:jl, ISBN:0198506732 Also known as: capZ binding, beta-actinin binding Relationships: is a type of GO:0008092 Subtypes: alpha-actinin binding [GO:0051393]